chondrocyte hypertrophy [GO:0003415] (biological process) Sources: GOC:ascb_2009, GOC:dph, GOC:tb Definition: The growth of a chondrocyte, where growth contributes to the progression of the chondrocyte over time. Regulation: RO_0002211 by regulation of chondrocyte hypertrophy [GO:1903041]; negatively regulated by negative regulation of chondrocyte hypertrophy [GO:1903042]; positively regulated by positive regulation of chondrocyte hypertrophy [GO:1903043] Relationships: is a type of GO:0048588; is part of chondrocyte development [GO:0002063] Subtypes: growth plate cartilage chondrocyte growth [GO:0003430]